{
  "gene_name": "Keratin-associated protein 9-1",
  "term_label": "Unknown molecular function",
  "term_id": "UNKNOWN:0001",
  "gene": "UniProtKB:A8MXZ3",
  "gene_symbol": "KRTAP9-1"
}